{
  "gene": "UniProtKB:Q15113",
  "term_id": "GO:0016504",
  "gene_symbol": "PCOLCE",
  "gene_name": "Procollagen C-endopeptidase enhancer 1",
  "term_label": "peptidase activator activity"
}